{
  "term_label": "axon",
  "gene": "UniProtKB:P63261",
  "term_id": "GO:0030424",
  "gene_symbol": "ACTG1",
  "gene_name": "Actin, cytoplasmic 2"
}